response to cycloalkane [GO:0014071] (biological process) Definition: Any process that results in a change in state or activity of a cell or an organism (in terms of movement, secretion, enzyme production, gene expression, etc.) as a result of a cycloalkane stimulus. A cycloalkane is a cyclic saturated hydrocarbon having the general formula CnH2n. Sources: GOC:ef Relationships: is a type of GO:0042221 Subtypes: cellular response to cycloalkane [GO:0071408] Regulation: regulated by regulation of response to cycloalkane [GO:1901431]; negatively regulated by GO:1901432; positively regulated by positive regulation of response to cycloalkane [GO:1901433]